{
  "gene_symbol": "MCM3",
  "gene_name": "DNA replication licensing factor MCM3",
  "term_label": "DNA strand elongation involved in DNA replication",
  "term_id": "GO:0006271",
  "gene": "UniProtKB:P25205"
}